{
  "gene": "UniProtKB:Q9H3T3",
  "gene_name": "Semaphorin-6B",
  "term_label": "chemorepellent activity",
  "gene_symbol": "SEMA6B",
  "term_id": "GO:0045499"
}